{
  "gene_symbol": "DDX39B",
  "term_label": "mRNA binding",
  "gene": "UniProtKB:Q13838",
  "term_id": "GO:0003729",
  "gene_name": "Spliceosome RNA helicase DDX39B"
}